{
  "term_label": "potassium channel regulator activity",
  "gene": "UniProtKB:Q9BQ31",
  "term_id": "GO:0015459",
  "gene_name": "Potassium voltage-gated channel subfamily S member 3",
  "gene_symbol": "KCNS3"
}